protein autophosphorylation [GO:0046777] (biological process) Regulation: regulated by GO:0031952; negatively regulated by negative regulation of protein autophosphorylation [GO:0031953]; RO_0002213 by positive regulation of protein autophosphorylation [GO:0031954] Relationships: is a type of protein phosphorylation [GO:0006468] Definition: The phosphorylation by a protein of one or more of its own amino acid residues (cis-autophosphorylation), or residues on an identical protein (trans-autophosphorylation). Also known as: protein amino acid autophosphorylation Subtypes: peptidyl-serine autophosphorylation [GO:0036289], protein trans-autophosphorylation [GO:0036290], peptidyl-tyrosine autophosphorylation [GO:0038083], peptidyl-threonine autophosphorylation [GO:1990443], peptidyl-aspartic acid autophosphorylation [GO:1990938] Sources: ISBN:0198506732